{
  "term_label": "Unknown biological process",
  "term_id": "UNKNOWN:0002",
  "gene_name": "Protein chibby homolog 3",
  "gene_symbol": "CBY3",
  "gene": "UniProtKB:A6NI87"
}